{
  "term_id": "UNKNOWN:0001",
  "gene": "UniProtKB:Q86YL5",
  "gene_name": "Testis development-related protein",
  "term_label": "Unknown molecular function",
  "gene_symbol": "TDRP"
}